{
  "gene": "UniProtKB:Q0P140",
  "term_label": "Unknown biological process",
  "gene_symbol": "HSD52",
  "gene_name": "Putative uncharacterized protein HSD52",
  "term_id": "UNKNOWN:0002"
}